purine ribonucleoside diphosphate biosynthetic process [GO:0009180] (biological process) Relationships: is a type of GO:0009136; is a type of purine ribonucleoside diphosphate metabolic process [GO:0009179]; is a type of GO:0009188 Subtypes: ADP biosynthetic process [GO:0006172], IDP biosynthetic process [GO:0046708], GDP biosynthetic process [GO:0046711] Sources: GOC:go_curators, ISBN:0198506732 Definition: The chemical reactions and pathways resulting in the formation of purine ribonucleoside diphosphate, a compound consisting of a purine base linked to a ribose sugar esterified with diphosphate on the sugar. Also known as: purine ribonucleoside diphosphate anabolism, purine ribonucleoside diphosphate biosynthesis, purine ribonucleoside diphosphate formation, purine ribonucleoside diphosphate synthesis